{
  "gene_name": "Double-stranded RNA-binding protein Staufen homolog 2",
  "gene": "UniProtKB:Q9NUL3",
  "term_label": "mRNA binding",
  "gene_symbol": "STAU2",
  "term_id": "GO:0003729"
}